polynucleotide 5' dephosphorylation [GO:0098507] (biological process) Sources: GOC:dos Definition: The process of removing one or more phosphate groups from the 5' end of a polynucleotide. Relationships: is a type of nucleobase-containing compound metabolic process [GO:0006139]; is_a GO:0016311; is a type of macromolecule metabolic process [GO:0043170]